{
  "term_id": "UNKNOWN:0001",
  "gene_symbol": "C1QTNF7",
  "gene_name": "Complement C1q tumor necrosis factor-related protein 7",
  "term_label": "Unknown molecular function",
  "gene": "UniProtKB:Q9BXJ2"
}